{
  "gene_name": "High affinity nerve growth factor receptor",
  "term_id": "GO:0030424",
  "term_label": "axon",
  "gene": "UniProtKB:P04629",
  "gene_symbol": "NTRK1"
}